rRNA (adenine-N6-)-methyltransferase activity [GO:0008988] (molecular function) Relationships: is a type of GO:0008170; is a type of rRNA (adenine) methyltransferase activity [GO:0016433] Subtypes: 23S rRNA (adenine(2030)-N(6))-methyltransferase activity [GO:0036307], GO:0052907, 23S rRNA (adenine(2085)-N(6))-dimethyltransferase activity [GO:0052910] Sources: RHEA:58728 Definition: Catalysis of the reaction: adenosine in rRNA + S-adenosyl-L-methionine = H+ + N(6)-methyladenosine in rRNA + S-adenosyl-L-homocysteine. Also known as: ErmC 23S rRNA methyltransferase, gene ksgA methyltransferase, S-adenosyl-L-methionine:rRNA (adenine-6-N-)-methyltransferase activity, S-adenosyl-L-methionine:rRNA (adenine-N6-)-methyltransferase activity, ribonucleic acid-adenine (N(6)) methylase activity, ribonucleic acid-adenine (N6) methylase activity, ribosomal ribonucleate adenine 6-methyltransferase activity